response to zinc ion [GO:0010043] (BP) Also known as: response to zinc Sources: GOC:sm Relationships: is a type of GO:0010038 Definition: Any process that results in a change in state or activity of a cell or an organism (in terms of movement, secretion, enzyme production, gene expression, etc.) as a result of a zinc ion stimulus. Subtypes: cellular response to zinc ion [GO:0071294], GO:1990359